{
  "gene_name": "Fibroblast growth factor 2",
  "term_label": "positive regulation of MAPK cascade",
  "gene": "UniProtKB:P09038",
  "gene_symbol": "FGF2",
  "term_id": "GO:0043410"
}